arginine N-methyltransferase activity [GO:0016273] (MF) Relationships: is a type of N-methyltransferase activity [GO:0008170]; is a type of GO:0008757 Sources: GOC:mah Definition: Enables the transfer of a methyl group from S-adenosyl-L-methionine to an amino group of an arginine residue. Subtypes: protein-arginine N-methyltransferase activity [GO:0016274]